{
  "term_id": "GO:0005634",
  "gene": "UniProtKB:P78396",
  "term_label": "nucleus",
  "gene_symbol": "CCNA1",
  "gene_name": "Cyclin-A1"
}